{
  "gene_symbol": "SIK2",
  "term_label": "cytoplasm",
  "term_id": "GO:0005737",
  "gene": "UniProtKB:Q9H0K1",
  "gene_name": "Serine_threonine-protein kinase SIK2"
}